SRP-dependent cotranslational protein targeting to membrane, docking [GO:0006615] (biological process) Also known as: SRP-dependent cotranslational membrane targeting, docking, SRP-dependent cotranslational protein-membrane targeting, docking, protein docking during SRP-dependent cotranslational protein targeting to membrane Definition: The process in which an SRP-bound ribosome forms a complex with the SRP receptor in the ER membrane, allowing the ribosome to bind to the membrane, during cotranslational membrane targeting. Sources: ISBN:0815316194 Relationships: is a type of protein to membrane docking [GO:0022615]; is part of SRP-dependent cotranslational protein targeting to membrane [GO:0006614]